{
  "gene_name": "Serine_threonine kinase-like domain-containing protein STKLD1",
  "gene": "UniProtKB:Q8NE28",
  "term_id": "GO:0004674",
  "term_label": "protein serine/threonine kinase activity",
  "gene_symbol": "STKLD1"
}